regulation of photoreceptor cell differentiation [GO:0046532] (biological process) Relationships: is a type of GO:0045664; regulates photoreceptor cell differentiation [GO:0046530] Definition: Any process that modulates the frequency, rate or extent of photoreceptor cell differentiation. An example of this process is found in Drosophila melanogaster. Also known as: regulation of photoreceptor differentiation Sources: GOC:go_curators Subtypes: regulation of eye photoreceptor cell development [GO:0042478], negative regulation of photoreceptor cell differentiation [GO:0046533], positive regulation of photoreceptor cell differentiation [GO:0046534], GO:0060224, regulation of compound eye photoreceptor cell differentiation [GO:0110116]